{
  "term_label": "plasma membrane",
  "term_id": "GO:0005886",
  "gene": "UniProtKB:Q8IY33",
  "gene_symbol": "MICALL2",
  "gene_name": "MICAL-like protein 2"
}